{
  "gene": "UniProtKB:P69905",
  "gene_name": "Hemoglobin subunit alpha",
  "term_label": "haptoglobin-hemoglobin complex",
  "term_id": "GO:0031838",
  "gene_symbol": "HBA2"
}